{
  "term_id": "GO:0042287",
  "gene_symbol": "MARCHF1",
  "gene": "UniProtKB:Q8TCQ1",
  "term_label": "MHC protein binding",
  "gene_name": "E3 ubiquitin-protein ligase MARCHF1"
}